{
  "gene_name": "Serine_threonine-protein kinase TAO1",
  "gene_symbol": "TAOK1",
  "term_label": "positive regulation of JNK cascade",
  "term_id": "GO:0046330",
  "gene": "UniProtKB:Q7L7X3"
}